{
  "gene_symbol": "VSTM5",
  "term_label": "positive regulation of excitatory synapse assembly",
  "gene_name": "V-set and transmembrane domain-containing protein 5",
  "gene": "UniProtKB:A8MXK1",
  "term_id": "GO:1904891"
}